{
  "gene_symbol": "CYP4V2",
  "gene_name": "Cytochrome P450 4V2",
  "term_id": "UNKNOWN:0003",
  "gene": "UniProtKB:Q6ZWL3",
  "term_label": "Unknown cellular component"
}